{
  "term_label": "Unknown biological process",
  "gene": "UniProtKB:Q86XR8",
  "gene_symbol": "CEP57",
  "gene_name": "Centrosomal protein of 57 kDa",
  "term_id": "UNKNOWN:0002"
}